{
  "term_label": "Unknown biological process",
  "term_id": "UNKNOWN:0002",
  "gene": "UniProtKB:Q6UX68",
  "gene_symbol": "XKR5",
  "gene_name": "XK-related protein 5"
}